{
  "gene": "UniProtKB:E9PB15",
  "gene_name": "Putative protein PTGES3L",
  "term_id": "GO:0051879",
  "gene_symbol": "PTGES3L",
  "term_label": "Hsp90 protein binding"
}